{
  "gene_symbol": "PIK3R5",
  "gene_name": "Phosphoinositide 3-kinase regulatory subunit 5",
  "term_id": "GO:0005942",
  "term_label": "phosphatidylinositol 3-kinase complex",
  "gene": "UniProtKB:Q8WYR1"
}